{
  "gene_symbol": "GALNT6",
  "term_id": "GO:0005794",
  "gene_name": "Polypeptide N-acetylgalactosaminyltransferase 6",
  "term_label": "Golgi apparatus",
  "gene": "UniProtKB:Q8NCL4"
}